{
  "gene_name": "Caspase-14",
  "term_id": "GO:0005737",
  "term_label": "cytoplasm",
  "gene": "UniProtKB:P31944",
  "gene_symbol": "CASP14"
}